{
  "gene_symbol": "BMP4",
  "term_label": "BMP signaling pathway",
  "gene": "UniProtKB:P12644",
  "term_id": "GO:0030509",
  "gene_name": "Bone morphogenetic protein 4"
}